{
  "gene_symbol": "EXOSC6",
  "gene": "UniProtKB:Q5RKV6",
  "term_label": "poly(A)-dependent snoRNA 3'-end processing",
  "term_id": "GO:0071051",
  "gene_name": "Exosome complex component MTR3"
}